diphosphoinositol pentakisphosphate 5-kinase activity [GO:0033200] (MF) Definition: Catalysis of the reaction: ATP + 4-diphospho-1D-myo-inositol (1,2,3,5,6)pentakisphosphate = ADP + 4,5-bisdiphosphoinositol-1D-myo-inositol (1,2,3,6)tetrakisphosphate, and ATP + 6-diphospho-1D-myo-inositol (1,2,3,4,5)pentakisphosphate = ADP + 5,6-bisdiphosphoinositol-1D-myo-inositol (1,2,3,4)tetrakisphosphate. References: PMID:17412958 Also known as: IP7 5-kinase activity, diphosphoinositol-pentakisphosphate 5-kinase activity, inositol heptakisphosphate 5-kinase activity Relationships: is a type of diphosphoinositol pentakisphosphate kinase activity [GO:0000829]